{
  "gene_name": "Perilipin-3",
  "term_id": "GO:0005829",
  "gene_symbol": "PLIN3",
  "term_label": "cytosol",
  "gene": "UniProtKB:O60664"
}